{
  "gene_name": "Beta-1,4-galactosyltransferase 5",
  "gene_symbol": "B4GALT5",
  "term_id": "GO:0005794",
  "gene": "UniProtKB:O43286",
  "term_label": "Golgi apparatus"
}